{
  "gene_symbol": "TSEN54",
  "term_label": "tRNA-type intron splice site recognition and cleavage",
  "gene": "UniProtKB:Q7Z6J9",
  "gene_name": "tRNA-splicing endonuclease subunit Sen54",
  "term_id": "GO:0000379"
}